{
  "gene_name": "Hexokinase HKDC1",
  "gene_symbol": "HKDC1",
  "term_label": "glucose 6-phosphate metabolic process",
  "term_id": "GO:0051156",
  "gene": "UniProtKB:Q2TB90"
}